rhamnose transmembrane transporter activity [GO:0015153] (molecular function) Definition: Enables the transfer of rhamnose from one side of a membrane to the other. Rhamnose occurs commonly as a compound of plant glycosides, in polysaccharides of gums and mucilages, and in bacterial polysaccharides. It is also a component of some plant cell wall polysaccharides and frequently acts as the sugar components of flavonoids. Relationships: is a type of hexose transmembrane transporter activity [GO:0015149]; is part of GO:0015762 Subtypes: rhamnose:proton symporter activity [GO:0015561] Also known as: ATP-dependent rhamnose transmembrane transporter activity, ATPase-coupled rhamnose transmembrane transporter activity, rhamnose-transporting ATPase activity Sources: GOC:ai, GOC:mtg_transport, ISBN:0815340729